{
  "gene_symbol": "MEGF10",
  "gene": "UniProtKB:Q96KG7",
  "term_label": "myoblast migration",
  "gene_name": "Multiple epidermal growth factor-like domains protein 10",
  "term_id": "GO:0051451"
}